{
  "gene_name": "Zinc finger protein 860",
  "term_label": "RNA polymerase II cis-regulatory region sequence-specific DNA binding",
  "gene_symbol": "ZNF860",
  "term_id": "GO:0000978",
  "gene": "UniProtKB:A6NHJ4"
}